{
  "term_id": "GO:0000045",
  "gene": "UniProtKB:Q9UMX0",
  "gene_symbol": "UBQLN1",
  "gene_name": "Ubiquilin-1",
  "term_label": "autophagosome assembly"
}